{
  "term_id": "GO:0030388",
  "gene": "UniProtKB:P08237",
  "term_label": "fructose 1,6-bisphosphate metabolic process",
  "gene_symbol": "PFKM",
  "gene_name": "ATP-dependent 6-phosphofructokinase, muscle type"
}